{
  "gene_name": "POU domain, class 6, transcription factor 2",
  "gene": "UniProtKB:P78424",
  "gene_symbol": "POU6F2",
  "term_label": "RNA polymerase II cis-regulatory region sequence-specific DNA binding",
  "term_id": "GO:0000978"
}